sex-specific pigmentation [GO:0048071] (biological process) Definition: Establishment of a pattern of pigment in one sex that is not observed in the other sex. Relationships: is a type of developmental process involved in reproduction [GO:0003006]; is a type of developmental pigmentation [GO:0048066]; is part of sex differentiation [GO:0007548] Sources: GOC:jid Subtypes: male pigmentation [GO:0048094], GO:0048095